{
  "gene_symbol": "RAB3C",
  "gene": "UniProtKB:Q96E17",
  "term_label": "plasma membrane",
  "term_id": "GO:0005886",
  "gene_name": "Ras-related protein Rab-3C"
}